{
  "term_id": "GO:0035493",
  "term_label": "SNARE complex assembly",
  "gene": "UniProtKB:P63027",
  "gene_symbol": "VAMP2",
  "gene_name": "Vesicle-associated membrane protein 2"
}